membrane fusion involved in acrosome reaction [GO:0002078] (biological process) Definition: The fusion of the plasma membrane of the sperm with the outer acrosomal membrane. Also known as: membrane fusion involved in the acrosomal reaction Relationships: is a type of cellular process involved in reproduction in multicellular organism [GO:0022412]; is a type of membrane fusion [GO:0061025]; is part of acrosome reaction [GO:0007340] References: PMID:3886029 Sources: GOC:dph